{
  "gene": "UniProtKB:O14576",
  "term_id": "GO:0010970",
  "term_label": "transport along microtubule",
  "gene_symbol": "DYNC1I1",
  "gene_name": "Cytoplasmic dynein 1 intermediate chain 1"
}